{
  "gene": "UniProtKB:Q68DN1",
  "gene_name": "Uncharacterized protein C2orf16",
  "term_id": "UNKNOWN:0001",
  "term_label": "Unknown molecular function",
  "gene_symbol": "C2orf16"
}